{
  "gene": "UniProtKB:O60478",
  "gene_symbol": "GPR137B",
  "term_label": "regulation of autophagy",
  "gene_name": "Integral membrane protein GPR137B",
  "term_id": "GO:0010506"
}